{
  "gene": "UniProtKB:O60812",
  "term_label": "nucleus",
  "gene_symbol": "HNRNPCL1",
  "gene_name": "Heterogeneous nuclear ribonucleoprotein C-like 1",
  "term_id": "GO:0005634"
}